metanephric renal vesicle induction [GO:0072094] (biological process) Relationships: is a type of renal vesicle induction [GO:0072034]; is a type of positive regulation of metanephros development [GO:0072216]; positively regulates metanephric renal vesicle formation [GO:0072093] Also known as: positive regulation of metanephros formation Sources: GOC:mtg_kidney_jan10 Definition: Signaling at short range between cells of the ureteric bud terminus and the kidney mesenchyme that positively regulates the formation of the metanephric renal vesicle.